{
  "term_id": "GO:0001755",
  "gene_symbol": "PHACTR4",
  "gene": "UniProtKB:Q8IZ21",
  "term_label": "neural crest cell migration",
  "gene_name": "Phosphatase and actin regulator 4"
}